vitamin B6 binding [GO:0070279] (molecular function) Subtypes: pyridoxal phosphate binding [GO:0030170], pyridoxal binding [GO:0070280], pyridoxamine binding [GO:0070281], pyridoxine binding [GO:0070282] Relationships: is a type of vitamin binding [GO:0019842]; is a type of heterocyclic compound binding [GO:1901363] Definition: Binding to a vitamin B6 compound: pyridoxal, pyridoxamine, pyridoxine, or the active form, pyridoxal phosphate. Sources: GOC:mah